{
  "gene": "UniProtKB:Q03188",
  "term_id": "GO:0019237",
  "gene_symbol": "CENPC",
  "gene_name": "Centromere protein C",
  "term_label": "centromeric DNA binding"
}